{
  "term_id": "UNKNOWN:0003",
  "term_label": "Unknown cellular component",
  "gene_symbol": "C17orf50",
  "gene_name": "Uncharacterized protein C17orf50",
  "gene": "UniProtKB:Q8WW18"
}